{
  "gene_symbol": "KRT33B",
  "term_label": "structural constituent of skin epidermis",
  "gene_name": "Keratin, type I cuticular Ha3-II",
  "gene": "UniProtKB:Q14525",
  "term_id": "GO:0030280"
}